{
  "gene_name": "Roquin-1",
  "gene": "UniProtKB:Q5TC82",
  "term_label": "double-stranded RNA binding",
  "term_id": "GO:0003725",
  "gene_symbol": "RC3H1"
}